{
  "term_id": "GO:0004534",
  "gene": "UniProtKB:Q8IZH2",
  "gene_symbol": "XRN1",
  "gene_name": "5'-3' exoribonuclease 1",
  "term_label": "5'-3' RNA exonuclease activity"
}